{
  "gene": "UniProtKB:Q9BU23",
  "term_id": "UNKNOWN:0001",
  "gene_name": "Lipase maturation factor 2",
  "gene_symbol": "LMF2",
  "term_label": "Unknown molecular function"
}